(S)-usnate reductase activity [GO:0046998] (molecular function) Definition: Catalysis of the reaction: (6R)-2-acetyl-6-(3-acetyl-2,4,6-trihydroxy-5-methylphenyl)-3-hydroxy-6-methylcyclohexa-2,4-dien-1-one + NAD+ = (S)-usnate + 2 H+ + NADH. Sources: EC:1.1.1.199, RHEA:21876 Also known as: L-usnic acid dehydrogenase activity, reduced-(S)-usnate:NAD+ oxidoreductase (ether-bond-forming) Relationships: is_a GO:0016616